{
  "gene_name": "Cullin-5",
  "gene": "UniProtKB:Q93034",
  "gene_symbol": "CUL5",
  "term_label": "ubiquitin protein ligase binding",
  "term_id": "GO:0031625"
}